{
  "gene_symbol": "TRAF3IP1",
  "gene": "UniProtKB:Q8TDR0",
  "gene_name": "TRAF3-interacting protein 1",
  "term_label": "Unknown molecular function",
  "term_id": "UNKNOWN:0001"
}